{
  "term_label": "Unknown cellular component",
  "gene": "UniProtKB:Q5I0X7",
  "gene_name": "Tetratricopeptide repeat protein 32",
  "term_id": "UNKNOWN:0003",
  "gene_symbol": "TTC32"
}